{
  "term_id": "UNKNOWN:0001",
  "gene": "UniProtKB:P61923",
  "gene_name": "Coatomer subunit zeta-1",
  "gene_symbol": "COPZ1",
  "term_label": "Unknown molecular function"
}